{
  "gene": "UniProtKB:Q6DKI7",
  "gene_name": "Transmembrane protein PVRIG",
  "term_id": "GO:0038023",
  "gene_symbol": "PVRIG",
  "term_label": "signaling receptor activity"
}